granulocyte macrophage colony-stimulating factor complex binding [GO:0042021] (molecular function) Relationships: is a type of cytokine binding [GO:0019955] Definition: Binding to a granulocyte macrophage colony-stimulating factor complex. Also known as: GM-CSF complex binding, GMC-SF complex binding, granulocyte macrophage colony stimulating factor complex binding Sources: GOC:ai